{
  "gene_name": "A-kinase anchor protein 1, mitochondrial",
  "term_id": "UNKNOWN:0002",
  "term_label": "Unknown biological process",
  "gene": "UniProtKB:Q92667",
  "gene_symbol": "AKAP1"
}